{
  "gene": "UniProtKB:P0DJD1",
  "gene_name": "RANBP2-like and GRIP domain-containing protein 2",
  "term_id": "GO:0019789",
  "gene_symbol": "RGPD2",
  "term_label": "SUMO transferase activity"
}